protein sulfation [GO:0006477] (biological process) Sources: GOC:curators Relationships: is a type of protein modification process [GO:0036211]; is a type of GO:0051923 Also known as: protein amino acid sulfation, protein amino acid sulphation Definition: The addition of a sulfate group as an ester to a protein amino acid. Subtypes: peptidyl-tyrosine sulfation [GO:0006478]